{
  "term_id": "GO:1990756",
  "term_label": "ubiquitin-like ligase-substrate adaptor activity",
  "gene_symbol": "KLHL2",
  "gene_name": "Kelch-like protein 2",
  "gene": "UniProtKB:O95198"
}